eiF2alpha phosphorylation in response to endoplasmic reticulum stress [GO:0036492] (BP) Relationships: is a type of regulation of translational initiation by eIF2 alpha phosphorylation [GO:0010998]; is a type of GO:0036491 Definition: The addition of a phosphate group on to the translation initiation factor eIF2alpha, as a result of endoplasmic reticulum stress. Also known as: eiF2alpha phosphorylation in response to ER stress, regulation of translation initiation by eiF2alpha phosphorylation in response to endoplasmic reticulum stress References: PMID:14676213, PMID:16835242 Sources: GOC:PARL, GOC:bf Regulation: regulated by regulation of endoplasmic reticulum stress-induced eIF2 alpha phosphorylation [GO:0060734]; negatively regulated by negative regulation of endoplasmic reticulum stress-induced eIF2 alpha phosphorylation [GO:1903912]